{
  "gene_name": "Forkhead box protein D3",
  "gene": "UniProtKB:Q9UJU5",
  "gene_symbol": "FOXD3",
  "term_id": "UNKNOWN:0003",
  "term_label": "Unknown cellular component"
}